{
  "term_label": "immunoglobulin complex",
  "term_id": "GO:0019814",
  "gene_symbol": "IGLV1-36",
  "gene_name": "Immunoglobulin lambda variable 1-36",
  "gene": "UniProtKB:A0A0B4J1U3"
}